{
  "gene_symbol": "IL12A",
  "gene": "UniProtKB:P29459",
  "term_label": "interleukin-12-mediated signaling pathway",
  "gene_name": "Interleukin-12 subunit alpha",
  "term_id": "GO:0035722"
}